positive regulation of pancreatic amylase secretion by cholecystokinin signaling pathway [GO:1902279] (biological process) Definition: A cholecystokinin signaling pathway that results in positive regulation of pancreatic amylase secretion. References: PMID:19028687 Sources: GOC:TermGenie, GOC:jc Relationships: is_a cholecystokinin signaling pathway [GO:0038188]; is a type of GO:1902278 Also known as: CCK-induced amylase release in pancreatic cell, CCK-mediated pancreatic amylase secretion, CCK-stimulated pancreatic amylase release, cholecystokinin-mediated pancreatic amylase secretion, up regulation of pancreatic amylase secretion by cholecystokinin signaling pathway, up-regulation of pancreatic amylase secretion by cholecystokinin signaling pathway, upregulation of pancreatic amylase secretion by cholecystokinin signaling pathway, activation of pancreatic amylase secretion by cholecystokinin signaling pathway